{
  "term_id": "GO:0004984",
  "gene_name": "Olfactory receptor 4L1",
  "gene_symbol": "OR4L1",
  "term_label": "olfactory receptor activity",
  "gene": "UniProtKB:Q8NH43"
}